regulation of dehydroaustinol biosynthetic process [GO:1900649] (BP) Sources: GOC:TermGenie, GOC:di Relationships: is a type of regulation of secondary metabolite biosynthetic process [GO:1900376]; regulates dehydroaustinol biosynthetic process [GO:1900563] Also known as: regulation of dehydroaustinol anabolism, regulation of dehydroaustinol biosynthesis, regulation of dehydroaustinol formation, regulation of dehydroaustinol synthesis Subtypes: negative regulation of dehydroaustinol biosynthetic process [GO:1900650], positive regulation of dehydroaustinol biosynthetic process [GO:1900651] Definition: Any process that modulates the frequency, rate or extent of dehydroaustinol biosynthetic process.